{
  "gene": "UniProtKB:Q6ZWT7",
  "gene_name": "Lysophospholipid acyltransferase 2",
  "gene_symbol": "MBOAT2",
  "term_id": "GO:0030258",
  "term_label": "lipid modification"
}